protein tyrosine phosphatase activity, metal-dependent [GO:0030946] (molecular function) Sources: GOC:mah Definition: Catalysis of the reaction: protein tyrosine phosphate + H2O = protein tyrosine + phosphate. This reaction requires metal ions. Relationships: is a type of protein tyrosine phosphatase activity [GO:0004725]